{
  "gene_name": "ATP-binding cassette sub-family C member 12",
  "gene": "UniProtKB:Q96J65",
  "term_id": "GO:0055085",
  "gene_symbol": "ABCC12",
  "term_label": "transmembrane transport"
}